{
  "gene": "UniProtKB:Q8N743",
  "gene_symbol": "KIR3DL3",
  "term_id": "GO:0004888",
  "term_label": "transmembrane signaling receptor activity",
  "gene_name": "Killer cell immunoglobulin-like receptor 3DL3"
}